XMP metabolic process [GO:0097292] (biological process) Sources: GOC:yaf Definition: The chemical reactions and pathways involving XMP, xanthosine monophosphate. Relationships: is a type of purine ribonucleotide metabolic process [GO:0009150]; is a type of GO:0009167 Subtypes: XMP biosynthetic process [GO:0097293] Also known as: XMP metabolism